{
  "gene_name": "Oligophrenin-1",
  "term_id": "GO:0030100",
  "gene_symbol": "OPHN1",
  "gene": "UniProtKB:O60890",
  "term_label": "regulation of endocytosis"
}